{
  "term_label": "cytoplasm",
  "term_id": "GO:0005737",
  "gene_symbol": "CHEK2",
  "gene": "UniProtKB:O96017",
  "gene_name": "Serine_threonine-protein kinase Chk2"
}